perikaryon [GO:0043204] (cellular component) Definition: The portion of the cell soma (neuronal cell body) that excludes the nucleus. Also known as: cell soma cytoplasm Sources: GOC:jl Relationships: is a type of GO:0110165; is part of neuronal cell body [GO:0043025]